{
  "gene_name": "Terminal uridylyltransferase 4",
  "gene_symbol": "TUT4",
  "gene": "UniProtKB:Q5TAX3",
  "term_id": "GO:0050265",
  "term_label": "RNA uridylyltransferase activity"
}